ciliary inversin compartment [GO:0097543] (cellular component) Definition: Proximal part of the ciliary shaft to which the inversin protein (also called Inv) specifically localizes. The inversin compartment appears to have a different protein composition than the rest of the cilium, although there is no structure that separates it form the distal part of the cilium. Relationships: is a type of cellular anatomical structure [GO:0110165]; is part of cilium [GO:0005929] Also known as: inversin compartment, Inv compartment of the cilium, cilial inversin compartment, cilium inversin compartment, flagellar inversin compartment, flagellum inversin compartment Note: Note that cilia and eukaryotic flagella are deemed to be equivalent. References: PMID:19050042 Sources: GOC:cilia